{
  "term_label": "transmembrane signaling receptor activity",
  "term_id": "GO:0004888",
  "gene_name": "Killer cell immunoglobulin-like receptor 3DL2",
  "gene": "UniProtKB:P43630",
  "gene_symbol": "KIR3DL2"
}